{
  "gene": "UniProtKB:Q15022",
  "gene_symbol": "SUZ12",
  "gene_name": "Polycomb protein SUZ12",
  "term_id": "GO:0035098",
  "term_label": "ESC/E(Z) complex"
}